{
  "gene_symbol": "ITGA3",
  "gene": "UniProtKB:P26006",
  "term_id": "GO:0007229",
  "gene_name": "Integrin alpha-3",
  "term_label": "integrin-mediated signaling pathway"
}